{
  "gene_symbol": "CRTC3",
  "gene_name": "CREB-regulated transcription coactivator 3",
  "term_id": "GO:0071878",
  "term_label": "negative regulation of adenylate cyclase-activating adrenergic receptor signaling pathway",
  "gene": "UniProtKB:Q6UUV7"
}